{
  "term_label": "vesicle docking",
  "term_id": "GO:0048278",
  "gene_symbol": "STX19",
  "gene": "UniProtKB:Q8N4C7",
  "gene_name": "Syntaxin-19"
}